2-methylbutanal reductase (NADPH) activity [GO:0032018] (molecular function) Definition: Catalysis of the reaction: 2-methylbutan-1-ol + NADP+ = 2-methylbutanal + NADPH + H+. Also known as: 2-methylbutanal reductase (NADP) activity, 2-methylbutanol:NADP oxidoreductase activity, 2-methylbutyraldehyde reductase (NADP) activity References: PMID:12210903 Sources: RHEA:84375 Relationships: is a type of alcohol dehydrogenase (NADP+) activity [GO:0008106]